large ribosomal subunit rRNA binding [GO:0070180] (molecular function) Definition: Binding to large ribosomal subunit RNA (LSU rRNA), a constituent of the large ribosomal subunit. In S. cerevisiae, this is the 25S rRNA. Also known as: 25S rRNA binding, LSU rRNA binding Relationships: is a type of rRNA binding [GO:0019843] Subtypes: GO:1990400 Sources: GOC:elh